DNA/DNA annealing activity [GO:1990814] (molecular function) References: PMID:22888405, PMID:25520186 Definition: An activity that facilitates the formation of a complementary double-stranded DNA molecule. Also known as: DNA reannealing activity Subtypes: ATP-dependent DNA/DNA annealing activity [GO:0036310] Relationships: is a type of GO:0003697; is_a catalytic activity, acting on DNA [GO:0140097]; is a type of annealing activity [GO:0140666]